alpha-mannosidase activity [GO:0004559] (molecular function) Also known as: 1,2-alpha-D-mannosidase activity, 1,2-alpha-mannosidase, p-nitrophenyl-alpha-mannosidase activity, alpha-D-mannopyranosidase activity, alpha-D-mannosidase activity, alpha-D-mannoside mannohydrolase activity, exo-alpha-mannosidase activity Definition: Catalysis of the hydrolysis of terminal, non-reducing alpha-D-mannose residues in alpha-D-mannosides. Sources: EC:3.2.1.24 Subtypes: glycoprotein endo-alpha-1,2-mannosidase activity [GO:0004569], mannan endo-1,6-alpha-mannosidase activity [GO:0008496], mannosyl-oligosaccharide mannosidase activity [GO:0015924], mannan 1,2-(1,3)-alpha-mannosidase activity [GO:0033915], mannan exo-1,2-1,6-alpha-mannosidase activity [GO:0033941], mannoside alpha-1,4-mannosidase activity [GO:0052766] Relationships: is a type of mannosidase activity [GO:0015923]